{
  "gene": "UniProtKB:P0DPI4",
  "gene_name": "T cell receptor beta diversity 1",
  "term_id": "UNKNOWN:0001",
  "gene_symbol": "TRBD1",
  "term_label": "Unknown molecular function"
}